{
  "term_id": "GO:0000785",
  "gene_symbol": "NSD1",
  "gene_name": "Histone-lysine N-methyltransferase, H3 lysine-36 specific",
  "term_label": "chromatin",
  "gene": "UniProtKB:Q96L73"
}